{
  "term_id": "UNKNOWN:0001",
  "gene_name": "WD repeat-containing protein 27",
  "gene": "UniProtKB:A2RRH5",
  "term_label": "Unknown molecular function",
  "gene_symbol": "WDR27"
}